monocyte differentiation [GO:0030224] (biological process) Also known as: monocyte cell differentiation Regulation: regulated by regulation of monocyte differentiation [GO:0045655]; negatively regulated by GO:0045656; positively regulated by positive regulation of monocyte differentiation [GO:0045657] Sources: GOC:mah Relationships: is a type of myeloid leukocyte differentiation [GO:0002573]; is a type of mononuclear cell differentiation [GO:1903131] Definition: The process in which a relatively unspecialized myeloid precursor cell acquires the specialized features of a monocyte.